{
  "gene_name": "Lymphocyte transmembrane adapter 1",
  "term_label": "plasma membrane",
  "gene_symbol": "LAX1",
  "gene": "UniProtKB:Q8IWV1",
  "term_id": "GO:0005886"
}